{
  "gene_name": "Mas-related G-protein coupled receptor member X3",
  "term_label": "G protein-coupled receptor activity",
  "gene_symbol": "MRGPRX3",
  "term_id": "GO:0004930",
  "gene": "UniProtKB:Q96LB0"
}